{
  "gene": "UniProtKB:Q96NL6",
  "gene_name": "Sodium channel and clathrin linker 1",
  "gene_symbol": "SCLT1",
  "term_id": "UNKNOWN:0001",
  "term_label": "Unknown molecular function"
}